{
  "term_id": "GO:0008173",
  "gene_symbol": "BCDIN3D",
  "gene_name": "RNA 5'-monophosphate methyltransferase",
  "term_label": "RNA methyltransferase activity",
  "gene": "UniProtKB:Q7Z5W3"
}